outer dynein arm docking complex [GO:0120228] (cellular component) Also known as: ODA docking complex, ODA-DC Definition: A complex which stabilizes the binding of and correctly positions the outer dynein arm complex along an A-tubule of the flagellar axoneme outer doublet microtubules. References: PMID:15064350, PMID:24067530, PMID:25192045, PMID:27486780, PMID:8045937 Sources: GOC:krc Relationships: is a type of protein-containing complex [GO:0032991]; is part of axoneme [GO:0005930]